L-carnitine CoA-transferase activity [GO:0008735] (molecular function) References: PMID:7815937, PMID:8188598 Also known as: L-carnitine dehydratase activity, L-carnitine hydro-lyase [4-(trimethylammonio)but-2-enoate-forming], L-carnitine hydro-lyase activity Relationships: is a type of CoA-transferase activity [GO:0008410] Definition: Catalysis of the reactions: (E)-4-(trimethylammonio)but-2-enoyl-CoA + L-carnitine = (E)-4-(trimethylammonio)but-2-enoate + L-carnitinyl-CoA and 4-trimethylammoniobutanoyl-CoA + L-carnitine = 4-trimethylammoniobutanoate + L-carnitinyl-CoA.